{
  "term_label": "nucleus",
  "gene": "UniProtKB:Q6P9F0",
  "term_id": "GO:0005634",
  "gene_name": "Coiled-coil domain-containing protein 62",
  "gene_symbol": "CCDC62"
}